positive regulation of cellular response to manganese ion [GO:1905804] (biological process) Relationships: is a type of positive regulation of cellular process [GO:0048522]; is a type of GO:0048584; is a type of regulation of cellular response to manganese ion [GO:1905802]; positively regulates cellular response to manganese ion [GO:0071287] Definition: Any process that activates or increases the frequency, rate or extent of cellular response to manganese ion. References: PMID:23721876 Sources: GOC:TermGenie, GO_REF:0000058 Also known as: positive regulation of cellular response to manganese, up regulation of cellular response to manganese, up regulation of cellular response to manganese ion, up-regulation of cellular response to manganese, up-regulation of cellular response to manganese ion, upregulation of cellular response to manganese, upregulation of cellular response to manganese ion, activation of cellular response to manganese, activation of cellular response to manganese ion